beta-aspartyl-N-acetylglucosaminidase activity [GO:0047406] (molecular function) Relationships: is_a hydrolase activity, hydrolyzing N-glycosyl compounds [GO:0016799] Also known as: 1-beta-aspartyl-N-acetyl-D-glucosaminylamine L-asparaginohydrolase activity, beta-aspartylacetylglucosaminidase activity Definition: Catalysis of the reaction: N(4)-(beta-N-acetyl-D-glucosaminyl)-L-asparagine + H2O = N-acetyl-D-glucosamine + L-asparagine. Sources: EC:3.2.2.11, RHEA:12324